{
  "gene": "UniProtKB:Q16629",
  "gene_name": "Serine_arginine-rich splicing factor 7",
  "gene_symbol": "SRSF7",
  "term_id": "GO:0016607",
  "term_label": "nuclear speck"
}